mitochondrial sulfate transmembrane transport [GO:1990557] (biological process) References: PMID:10428783 Definition: The process in which sulfate is transported across a mitochondrial membrane, into or out of the mitochondrion. Relationships: is a type of sulfate transmembrane transport [GO:1902358]